{
  "gene_symbol": "OR14A16",
  "term_id": "GO:0004984",
  "term_label": "olfactory receptor activity",
  "gene": "UniProtKB:Q8NHC5",
  "gene_name": "Olfactory receptor 14A16"
}